{
  "term_id": "GO:0005886",
  "gene": "UniProtKB:P42892",
  "term_label": "plasma membrane",
  "gene_symbol": "ECE1",
  "gene_name": "Endothelin-converting enzyme 1"
}